{
  "gene_name": "Retinol dehydrogenase 12",
  "gene": "UniProtKB:Q96NR8",
  "term_label": "Unknown molecular function",
  "term_id": "UNKNOWN:0001",
  "gene_symbol": "RDH12"
}